{
  "term_id": "GO:0005737",
  "gene_symbol": "DACT2",
  "gene": "UniProtKB:Q5SW24",
  "gene_name": "Dapper homolog 2",
  "term_label": "cytoplasm"
}